negative regulation of AV node cell action potential [GO:1903950] (biological process) Also known as: down regulation of AV node cardiac muscle cell action potential, down regulation of AV node cell action potential, down regulation of atrioventricular node cardiac muscle cell action potential, down-regulation of AV node cardiac muscle cell action potential, down-regulation of AV node cell action potential, down-regulation of atrioventricular node cardiac muscle cell action potential, downregulation of AV node cardiac muscle cell action potential, downregulation of AV node cell action potential, downregulation of atrioventricular node cardiac muscle cell action potential, negative regulation of AV node cardiac muscle cell action potential, negative regulation of atrioventricular node cardiac muscle cell action potential, inhibition of AV node cardiac muscle cell action potential, inhibition of AV node cell action potential, inhibition of atrioventricular node cardiac muscle cell action potential References: PMID:25281747 Sources: GOC:BHF, GOC:TermGenie, GOC:mtg_cardiac_conduct_nov11, GOC:nc, GO_REF:0000058 Definition: Any process that stops, prevents or reduces the frequency, rate or extent of AV node cell action potential. Relationships: is a type of negative regulation of action potential [GO:0045759]; is a type of GO:0098904; negatively regulates AV node cell action potential [GO:0086016]